{
  "gene_name": "Anosmin-1",
  "gene_symbol": "ANOS1",
  "gene": "UniProtKB:P23352",
  "term_id": "UNKNOWN:0001",
  "term_label": "Unknown molecular function"
}